{
  "term_id": "GO:0003723",
  "term_label": "RNA binding",
  "gene_name": "5'-3' exoribonuclease 2",
  "gene_symbol": "XRN2",
  "gene": "UniProtKB:Q9H0D6"
}